{
  "gene": "UniProtKB:Q9UPQ8",
  "term_id": "GO:0004168",
  "term_label": "dolichol kinase activity",
  "gene_symbol": "DOLK",
  "gene_name": "Dolichol kinase"
}